positive regulation of mesenchymal cell apoptotic process involved in metanephros development [GO:1900213] (biological process) References: PMID:17314325 Sources: GOC:TermGenie, GOC:mtg_apoptosis, GOC:mtg_kidney_jan10, GOC:yaf Relationships: is a type of regulation of mesenchymal cell apoptotic process involved in metanephros development [GO:1900211]; is a type of positive regulation of apoptotic process involved in development [GO:1904747]; is a type of positive regulation of mesenchymal cell apoptotic process [GO:2001055]; positively regulates mesenchymal cell apoptotic process involved in metanephros development [GO:1900200] Subtypes: positive regulation of mesenchymal cell apoptotic process involved in metanephric nephron morphogenesis [GO:0072306] Definition: Any process that activates or increases the frequency, rate or extent of mesenchymal cell apoptotic process involved in metanephros development. Also known as: up regulation of mesenchymal cell apoptosis involved in metanephros development, up-regulation of mesenchymal cell apoptosis involved in metanephros development, upregulation of mesenchymal cell apoptosis involved in metanephros development, activation of mesenchymal cell apoptosis involved in metanephros development, positive regulation of mesenchymal cell apoptosis involved in metanephros development